{
  "term_label": "wybutosine biosynthetic process",
  "gene": "UniProtKB:Q6NUM6",
  "gene_name": "S-adenosyl-L-methionine-dependent tRNA 4-demethylwyosine synthase TYW1B",
  "gene_symbol": "TYW1B",
  "term_id": "GO:0031591"
}